{
  "gene_name": "Putative uncharacterized protein PP632",
  "gene_symbol": "PP632",
  "term_id": "UNKNOWN:0001",
  "gene": "UniProtKB:Q6XCG6",
  "term_label": "Unknown molecular function"
}